{
  "gene_name": "Keratin-associated protein 9-7",
  "gene": "UniProtKB:A8MTY7",
  "term_id": "UNKNOWN:0002",
  "gene_symbol": "KRTAP9-7",
  "term_label": "Unknown biological process"
}